monosaccharide transmembrane transport [GO:0015749] (biological process) Definition: The process in which a monosaccharide is transported across a lipid bilayer, from one side of a membrane to the other. Monosaccharides are the simplest carbohydrates; they are polyhydric alcohols containing either an aldehyde or a keto group and between three to ten or more carbon atoms. They form the constitutional repeating units of oligo- and polysaccharides. Relationships: is a type of carbohydrate transmembrane transport [GO:0034219] Subtypes: GO:0008645, pentose transmembrane transport [GO:0015750], L-ascorbic acid transmembrane transport [GO:0015882], 2-keto-3-deoxygluconate transmembrane transport [GO:0046411] Sources: GOC:TermGenie, GOC:vw, GO_REF:0000069 Also known as: monosaccharide transport